{
  "gene_symbol": "RSPH10B2",
  "gene": "UniProtKB:B2RC85",
  "term_id": "UNKNOWN:0002",
  "gene_name": "Radial spoke head 10 homolog B2",
  "term_label": "Unknown biological process"
}